{
  "gene_symbol": "ANAPC2",
  "gene_name": "Anaphase-promoting complex subunit 2",
  "term_id": "GO:0070979",
  "term_label": "protein K11-linked ubiquitination",
  "gene": "UniProtKB:Q9UJX6"
}